tRNA transmembrane transporter activity [GO:0051034] (molecular function) Relationships: is a type of RNA transmembrane transporter activity [GO:0051033]; is part of tRNA transport [GO:0051031] Sources: GOC:ai Definition: Enables the transfer of tRNA, transfer ribonucleic acid, from one side of a membrane to the other.